{
  "gene": "UniProtKB:Q8TAM2",
  "gene_name": "Tetratricopeptide repeat protein 8",
  "gene_symbol": "TTC8",
  "term_label": "non-motile cilium",
  "term_id": "GO:0097730"
}